{
  "term_id": "GO:0005886",
  "gene": "UniProtKB:P63252",
  "term_label": "plasma membrane",
  "gene_symbol": "KCNJ2",
  "gene_name": "Inward rectifier potassium channel 2"
}